{
  "term_id": "GO:0007417",
  "term_label": "central nervous system development",
  "gene_name": "Macrophage-capping protein",
  "gene_symbol": "CAPG",
  "gene": "UniProtKB:P40121"
}